semaphorin-plexin signaling pathway involved in bone trabecula morphogenesis [GO:1900220] (biological process) Relationships: is a type of semaphorin-plexin signaling pathway [GO:0071526]; is part of bone trabecula morphogenesis [GO:0061430] Also known as: semaphorin-plexin signaling pathway of bone trabecula morphogenesis, semaphorin-plexin signalling pathway of bone trabecula morphogenesis Definition: Any semaphorin-plexin signaling pathway that contributes to bone trabecula morphogenesis. Sources: GOC:BHF, GOC:TermGenie